wound healing [GO:0042060] (biological process) Subtypes: wound healing involved in inflammatory response [GO:0002246] Definition: The series of events that restore integrity to a damaged tissue, following an injury. Regulation: regulated by regulation of wound healing [GO:0061041]; negatively regulated by negative regulation of wound healing [GO:0061045]; positively regulated by GO:0090303 References: PMID:15269788 Sources: GOC:bf Relationships: is a type of response to wounding [GO:0009611]; has part tissue regeneration [GO:0042246]